{
  "term_id": "GO:0005634",
  "gene_name": "Polyadenylate-binding protein 4",
  "gene": "UniProtKB:Q13310",
  "term_label": "nucleus",
  "gene_symbol": "PABPC4"
}